glucarate O-hydroxycinnamoyltransferase activity [GO:0047170] (molecular function) Definition: Catalysis of the reaction: D-glucarate + sinapoyl-CoA = 2-O-sinapoyl-D-glucarate + CoA. Relationships: is a type of O-hydroxycinnamoyltransferase activity [GO:0050737] Also known as: sinapoyl-CoA:glucarate O-(hydroxycinnamoyl)transferase activity Sources: EC:2.3.1.131, RHEA:23308